{
  "term_id": "GO:0007283",
  "gene_symbol": "NICOL1",
  "term_label": "spermatogenesis",
  "gene_name": "Neuropeptide-like protein C4orf48",
  "gene": "UniProtKB:Q5BLP8"
}